mesonephric glomerular mesangial cell differentiation [GO:0061259] (BP) Definition: The process in which relatively unspecialized cells acquire specialized structural and/or functional features that characterize the glomerular mesangial cells of the mesonephros as it progresses from its formation to the mature state. Relationships: is a type of mesonephric mesangial cell differentiation [GO:0061260]; is a type of glomerular mesangial cell differentiation [GO:0072008]; BFO_0000050 mesonephric glomerular mesangium development [GO:0061247] Sources: GOC:mtg_kidney_jan10